positive regulation of interleukin-4 production [GO:0032753] (biological process) Definition: Any process that activates or increases the frequency, rate, or extent of interleukin-4 production. Relationships: is a type of positive regulation of cytokine production [GO:0001819]; is a type of GO:0032673; RO_0002213 interleukin-4 production [GO:0032633] Sources: GOC:mah Also known as: positive regulation of IL-4 production, up regulation of interleukin-4 production, up-regulation of interleukin-4 production, upregulation of interleukin-4 production, activation of interleukin-4 production, positive regulation of interleukin-4 biosynthetic process, positive regulation of interleukin-4 secretion, stimulation of interleukin-4 production